{
  "gene_name": "CAP-Gly domain-containing linker protein 2",
  "gene": "UniProtKB:Q9UDT6",
  "term_id": "GO:0035371",
  "term_label": "microtubule plus-end",
  "gene_symbol": "CLIP2"
}